{
  "gene_name": "UBX domain-containing protein 4",
  "term_id": "GO:0005783",
  "gene_symbol": "UBXN4",
  "term_label": "endoplasmic reticulum",
  "gene": "UniProtKB:Q92575"
}